{
  "term_id": "GO:0033550",
  "gene_symbol": "DUSP6",
  "gene_name": "Dual specificity protein phosphatase 6",
  "gene": "UniProtKB:Q16828",
  "term_label": "MAP kinase tyrosine phosphatase activity"
}